{
  "term_label": "G protein-coupled peptide receptor activity",
  "gene_symbol": "SCTR",
  "gene_name": "Secretin receptor",
  "gene": "UniProtKB:P47872",
  "term_id": "GO:0008528"
}